{
  "gene_symbol": "CHRNB4",
  "gene_name": "Neuronal acetylcholine receptor subunit beta-4",
  "gene": "UniProtKB:P30926",
  "term_label": "synapse",
  "term_id": "GO:0045202"
}